{
  "gene_symbol": "SERPING1",
  "gene": "UniProtKB:P05155",
  "term_id": "GO:0005615",
  "term_label": "extracellular space",
  "gene_name": "Plasma protease C1 inhibitor"
}